{
  "gene_name": "Acyl-coenzyme A synthetase ACSM2A, mitochondrial",
  "gene_symbol": "ACSM2A",
  "term_id": "GO:0005759",
  "term_label": "mitochondrial matrix",
  "gene": "UniProtKB:Q08AH3"
}